growth plate cartilage chondrocyte proliferation [GO:0003419] (biological process) Regulation: regulated by regulation of growth plate cartilage chondrocyte proliferation [GO:0003420]; positively regulated by positive regulation of growth plate cartilage chondrocyte proliferation [GO:0061913]; negatively regulated by GO:0061914 Sources: GOC:ascb_2009, GOC:dph, GOC:tb Relationships: is a type of cell population proliferation [GO:0008283]; is part of GO:0003417 Definition: The multiplication or reproduction of chondrocytes in a growing endochondral bone, resulting in the expansion of a cell population.